{
  "gene_symbol": "KRT39",
  "term_label": "keratin filament",
  "gene": "UniProtKB:Q6A163",
  "gene_name": "Keratin, type I cytoskeletal 39",
  "term_id": "GO:0045095"
}